type IV pilus-dependent motility [GO:0043107] (biological process) Relationships: is a type of cell motility [GO:0048870] Also known as: TFP-dependent motility, TFP-dependent movement, type 4 pilus-dependent motility, type four pilus-dependent motility, social gliding motility, twitching motility References: PMID:12704238 Sources: GOC:go_curators Definition: Any process involved in the controlled movement of a bacterial cell which is dependent on the presence of type IV pili. Includes social gliding motility and twitching motility.